male meiosis sister chromatid cohesion [GO:0007065] (biological process) Relationships: is a type of GO:0051177 Definition: The joining of the sister chromatids of a replicated chromosome along the entire length of the chromosome that occurs during meiosis in a male. Sources: GOC:ai